{
  "term_label": "myofibril",
  "gene_symbol": "LMOD2",
  "gene": "UniProtKB:Q6P5Q4",
  "gene_name": "Leiomodin-2",
  "term_id": "GO:0030016"
}